{
  "gene": "UniProtKB:Q9C0H6",
  "gene_symbol": "KLHL4",
  "gene_name": "Kelch-like protein 4",
  "term_id": "GO:0043161",
  "term_label": "proteasome-mediated ubiquitin-dependent protein catabolic process"
}